{
  "term_id": "GO:0042981",
  "gene": "UniProtKB:D6R901",
  "gene_symbol": "USP17L21",
  "term_label": "regulation of apoptotic process",
  "gene_name": "Ubiquitin carboxyl-terminal hydrolase 17-like protein 21"
}